{
  "term_id": "GO:0016477",
  "gene_symbol": "SH3D21",
  "gene_name": "SH3 domain-containing protein 21",
  "gene": "UniProtKB:A4FU49",
  "term_label": "cell migration"
}